regulation of uredinium development [GO:0075280] (biological process) Relationships: is a type of regulation of spore-bearing organ development [GO:0075260]; regulates uredinium development [GO:0075279] Definition: Any process that modulates the frequency, rate or extent of uredinium development, a process that leads to the formation of a reddish, pustule-like structure formed by a rust fungus and consisting of uredospores. Sources: GOC:pamgo_curators Subtypes: positive regulation of uredinium development [GO:0075281], GO:0075282